{
  "gene_name": "Rho-related BTB domain-containing protein 2",
  "term_label": "regulation of cell shape",
  "gene": "UniProtKB:Q9BYZ6",
  "gene_symbol": "RHOBTB2",
  "term_id": "GO:0008360"
}